centromere-nuclear envelope anchor activity [GO:0140449] (molecular function) References: PMID:31635174 Also known as: centromere nuclear envelope anchor activity, centromere nuclear envelope tether activity, centromere-inner nuclear envelope anchor activity, centromere-inner nuclear envelope tether activity, chromosome, centromeric region-nuclear envelope anchor activity, nuclear envelope-centromere anchor activity, nuclear envelope-centromere tether activity Definition: The binding activity of a molecule that brings together the centromeric region of a chromosome and the inner nuclear membrane by interacting with both the centromere/kinetochore complex and the nuclear membrane, in order to establish and maintain the centromere/kinetochore location. Relationships: is a type of protein-membrane adaptor activity [GO:0043495]; is part of centromere clustering at the mitotic interphase nuclear envelope [GO:0072766]